positive regulation of positive chemotaxis to cAMP by DIF-1 [GO:0061126] (BP) Sources: GOC:dph Relationships: is a type of regulation of positive chemotaxis to cAMP by DIF-1 [GO:0061120]; is a type of positive regulation of positive chemotaxis to cAMP by chlorinated alkylphenone [GO:0061124] Definition: Any process that increases the rate, frequency, or extent of directed movement of a motile cell or organism up a concentration gradient of 3',5'-cAMP by the action of DIF-1. DIF-1 is a chlorinated alkylphenone.